cellular response to unfolded protein [GO:0034620] (BP) Note: Note that this term should not be confused with 'unfolded protein response ; GO:0030968', which refers to the signaling pathways that respond to the presence of unfolded proteins in the ER. Subtypes: mitochondrial unfolded protein response [GO:0034514] Definition: Any process that results in a change in state or activity of a cell (in terms of movement, secretion, enzyme production, gene expression, etc.) as a result of an unfolded protein stimulus. Relationships: is a type of GO:0006986; is a type of cellular response to topologically incorrect protein [GO:0035967] Sources: GOC:mah Also known as: heat shock protein activity